{
  "gene_name": "FAD synthase",
  "term_id": "GO:0006747",
  "gene": "UniProtKB:Q8NFF5",
  "gene_symbol": "FLAD1",
  "term_label": "FAD biosynthetic process"
}